amino-acid betaine transport [GO:0015838] (biological process) Subtypes: carnitine transport [GO:0015879], glycine betaine transport [GO:0031460], 4-(trimethylammonio)butanoate transport [GO:1900751] Definition: The directed movement of betaine, the N-trimethyl derivative of an amino acid, into, out of or within a cell, or between cells, by means of some agent such as a transporter or pore. Relationships: is_a quaternary ammonium group transport [GO:0015697]; is a type of modified amino acid transport [GO:0072337] Sources: GOC:ai Also known as: betaine transport